myosin XII complex [GO:0031482] (cellular component) References: PMID:10722873 Definition: A myosin complex containing one or more class XII myosin heavy chains and associated light chains; myosin XII contains a large tail region with two MyTH4 domains and a short region of coiled coil. Relationships: is a type of unconventional myosin complex [GO:0016461]